{
  "gene_name": "1-phosphatidylinositol 4,5-bisphosphate phosphodiesterase beta-1",
  "gene": "UniProtKB:Q9NQ66",
  "term_id": "GO:0048015",
  "term_label": "phosphatidylinositol-mediated signaling",
  "gene_symbol": "PLCB1"
}